{
  "gene": "UniProtKB:Q05481",
  "term_id": "GO:0000976",
  "term_label": "transcription cis-regulatory region binding",
  "gene_symbol": "ZNF91",
  "gene_name": "Zinc finger protein 91"
}